{
  "term_id": "GO:0016608",
  "gene_symbol": "GHRL",
  "term_label": "growth hormone-releasing hormone activity",
  "gene": "UniProtKB:Q9UBU3",
  "gene_name": "Appetite-regulating hormone"
}